cell-cell junction maintenance [GO:0045217] (BP) Definition: The maintenance of junctions between cells. Relationships: is a type of cell junction maintenance [GO:0034331]; is_a cell-cell junction organization [GO:0045216] Sources: GOC:ai Also known as: intercellular junction maintenance Subtypes: desmosome maintenance [GO:0002160], adherens junction maintenance [GO:0034334], paranodal junction maintenance [GO:1990227]